lipid-A-disaccharide synthase activity [GO:0008915] (molecular function) Also known as: UDP-2,3-bis(3-hydroxytetradecanoyl)glucosamine:2,3-bis-(3-hydroxytetradecanoyl)-beta-D-glucosaminyl-1-phosphate 2,3-bis(3-hydroxytetradecanoyl)-glucosaminyltransferase activity Relationships: is a type of UDP-glycosyltransferase activity [GO:0008194]; is a type of hexosyltransferase activity [GO:0016758] Definition: Catalysis of the reaction: a lipid X + a UDP-2-N,3-O-bis[(3R)-3-hydroxyacyl]-alpha-D-glucosamine = a lipid A disaccharide + UDP + H+. Sources: RHEA:67828